2-hydroxy-6-oxonona-2,4-dienedioate hydrolase activity [GO:0018771] (molecular function) Definition: Catalysis of the reaction: (2Z,4E)-2-hydroxy-6-oxonona-2,4-dienedioate + H2O = (2Z)-2-hydroxypenta-2,4-dienoate + H+ + succinate. Sources: RHEA:34187 Relationships: is a type of hydrolase activity, acting on acid carbon-carbon bonds, in ketonic substances [GO:0016823] Also known as: (2E,4Z)-2-hydroxy-6-oxona-2,4-dienedioate succinylhydrolase activity, 2-hydroxy-6-ketonona-2,4-dienedoic acid hydrolase activity